inositol diphosphate tetrakisphosphate diphosphatase activity [GO:0052840] (molecular function) Relationships: is a type of GO:0008486 Subtypes: inositol-5-diphosphate-1,3,4,6-tetrakisphosphate diphosphatase activity [GO:0106211] Definition: Catalysis of the reaction: diphospho-1D-myo-inositol tetrakisphosphate + H2O = 1D-myo-inositol pentakisphosphate + phosphate. References: PMID:10827188, PMID:11502751